{
  "gene_name": "Putative uncharacterized protein encoded by LINC00526",
  "gene": "UniProtKB:Q96FQ7",
  "term_id": "UNKNOWN:0003",
  "gene_symbol": "LINC00526",
  "term_label": "Unknown cellular component"
}